mRNA 5'-diphosphatase activity [GO:0034353] (molecular function) References: PMID:17612492, PMID:18202662 Sources: GOC:jh2 Also known as: RNA pyrophosphohydrolase activity Relationships: is a type of pyrophosphatase activity [GO:0016462]; is a type of catalytic activity, acting on RNA [GO:0140098] Definition: Catalysis of the removal of a 5' terminal diphosphate from the 5'-triphosphate end of an mRNA, leaving a 5'-monophosphate end.